{
  "gene_symbol": "SIMC1",
  "gene": "UniProtKB:Q8NDZ2",
  "gene_name": "SUMO-interacting motif-containing protein 1",
  "term_label": "Unknown biological process",
  "term_id": "UNKNOWN:0002"
}